{
  "gene": "UniProtKB:O43612",
  "gene_symbol": "HCRT",
  "term_label": "sleep",
  "term_id": "GO:0030431",
  "gene_name": "Hypocretin neuropeptide precursor"
}